{
  "gene_name": "Putative uncharacterized protein FLJ44790",
  "term_label": "Unknown cellular component",
  "gene": "UniProtKB:Q6ZTC4",
  "gene_symbol": "Q6ZTC4",
  "term_id": "UNKNOWN:0003"
}